{
  "gene_symbol": "C4A",
  "gene": "UniProtKB:P0C0L4",
  "term_id": "GO:0005615",
  "term_label": "extracellular space",
  "gene_name": "Complement C4-A"
}